positive regulation of emodin biosynthetic process [GO:1900666] (biological process) Relationships: is_a positive regulation of small molecule metabolic process [GO:0062013]; is a type of positive regulation of secondary metabolite biosynthetic process [GO:1900378]; is a type of regulation of emodin biosynthetic process [GO:1900664]; RO_0002213 GO:1900575 Definition: Any process that activates or increases the frequency, rate or extent of emodin biosynthetic process. Sources: GOC:TermGenie, GOC:di Also known as: activation of emodin anabolism, activation of emodin biosynthesis, activation of emodin formation, activation of emodin synthesis, positive regulation of emodin anabolism, positive regulation of emodin biosynthesis, positive regulation of emodin formation, positive regulation of emodin synthesis, up regulation of emodin anabolism, up regulation of emodin biosynthesis, up regulation of emodin biosynthetic process, up regulation of emodin formation, up regulation of emodin synthesis, up-regulation of emodin anabolism, up-regulation of emodin biosynthesis, up-regulation of emodin biosynthetic process, up-regulation of emodin formation, up-regulation of emodin synthesis, upregulation of emodin anabolism, upregulation of emodin biosynthesis, upregulation of emodin biosynthetic process, upregulation of emodin formation, upregulation of emodin synthesis, activation of emodin biosynthetic process